{
  "gene_symbol": "KIF5C",
  "term_id": "GO:0005737",
  "gene_name": "Kinesin heavy chain isoform 5C",
  "term_label": "cytoplasm",
  "gene": "UniProtKB:O60282"
}